{
  "gene": "UniProtKB:A0A1B0GTH9",
  "gene_symbol": "LOC100505841",
  "term_id": "UNKNOWN:0003",
  "gene_name": "Zinc finger protein 474",
  "term_label": "Unknown cellular component"
}